{
  "gene_symbol": "SNURF",
  "term_id": "UNKNOWN:0001",
  "term_label": "Unknown molecular function",
  "gene_name": "SNRPN upstream reading frame protein",
  "gene": "UniProtKB:Q9Y675"
}